flotillin complex [GO:0016600] (cellular component) Definition: A protein complex that contains flotillin-1 and flotillin-2, and may contain associated proteins. Flotillins associate into membrane microdomains resembling caveolae. References: PMID:17206938, PMID:17600709 Note: See also the cellular component term 'caveola ; GO:0005901'. Relationships: is a type of GO:0098797; is part of caveola [GO:0005901]